{
  "gene": "UniProtKB:O15303",
  "term_id": "GO:0007216",
  "gene_name": "Metabotropic glutamate receptor 6",
  "gene_symbol": "GRM6",
  "term_label": "G protein-coupled glutamate receptor signaling pathway"
}